inorganic anion import across plasma membrane [GO:0098658] (biological process) Also known as: inorganic anion import into cell Definition: The directed movement of inorganic anions from outside of a cell, across the plasma membrane and into the cytosol. Relationships: is_a inorganic anion transport [GO:0015698]; is a type of inorganic ion import across plasma membrane [GO:0099587] Subtypes: silicic acid import across plasma membrane [GO:0015708], sulfate import across plasma membrane [GO:1902434] Sources: GOC:dos